collagen type XXII trimer [GO:1990321] (cellular component) References: PMID:17876790 Relationships: is_a FACIT collagen trimer [GO:0005593] Definition: A collagen homotrimer of alpha1(XXII) chains; type XXII collagen triple helices acts as a cell adhesion ligand for skin epithelial cells and fibroblasts.